{
  "gene_name": "Rho GTPase-activating protein 4",
  "term_id": "GO:0007399",
  "gene_symbol": "ARHGAP4",
  "gene": "UniProtKB:P98171",
  "term_label": "nervous system development"
}